{
  "gene_name": "Neuronal acetylcholine receptor subunit beta-4",
  "term_id": "GO:0022848",
  "gene_symbol": "CHRNB4",
  "gene": "UniProtKB:P30926",
  "term_label": "acetylcholine-gated monoatomic cation-selective channel activity"
}